{
  "gene_symbol": "LRRC32",
  "term_label": "signaling receptor activity",
  "gene_name": "Transforming growth factor beta activator LRRC32",
  "term_id": "GO:0038023",
  "gene": "UniProtKB:Q14392"
}